L-cystine transmembrane transporter activity [GO:0015184] (molecular function) Definition: Enables the transfer of L-cystine from one side of a membrane to the other. Relationships: is_a sulfur amino acid transmembrane transporter activity [GO:0000099]; is a type of GO:0015179; is a type of modified amino acid transmembrane transporter activity [GO:0072349]; is part of L-cystine transport [GO:0015811] Sources: GOC:go_curators, GOC:mtg_transport, ISBN:0198506732, ISBN:0815340729 Also known as: L-cystine transporter activity, cystine/diaminopimelate porter activity